{
  "term_label": "Unknown cellular component",
  "gene_symbol": "LANCL1",
  "gene": "UniProtKB:O43813",
  "term_id": "UNKNOWN:0003",
  "gene_name": "Glutathione S-transferase LANCL1"
}